positive regulation of antibacterial peptide production [GO:0002803] (biological process) Definition: Any process that activates or increases the frequency, rate, or extent of antibacterial peptide production. Relationships: is a type of positive regulation of antimicrobial peptide production [GO:0002225]; is a type of regulation of antibacterial peptide production [GO:0002786]; is a type of positive regulation of defense response to bacterium [GO:1900426]; positively regulates GO:0002778 Subtypes: GO:0002799, positive regulation of antibacterial peptide biosynthetic process [GO:0006963] Sources: GOC:add Also known as: up regulation of antibacterial peptide production, up-regulation of antibacterial peptide production, upregulation of antibacterial peptide production, activation of antibacterial peptide production, stimulation of antibacterial peptide production